plastid outer membrane organization [GO:0009666] (biological process) Relationships: is a type of plastid membrane organization [GO:0009668] Sources: GOC:ai, GOC:dph, GOC:jl, GOC:mah Definition: A process that is carried out at the cellular level which results in the assembly, arrangement of constituent parts, or disassembly of the outer membrane of a plastid. Also known as: plastid outer membrane organisation, plastid outer membrane organization and biogenesis